carbohydrate derivative transmembrane transporter activity [GO:1901505] (molecular function) Sources: GOC:TermGenie, GOC:pr Subtypes: nucleoside transmembrane transporter activity [GO:0005337], nucleotide-sugar transmembrane transporter activity [GO:0005338], purine ribonucleotide transmembrane transporter activity [GO:0005346], hexose phosphate transmembrane transporter activity [GO:0015119], sialic acid transmembrane transporter activity [GO:0015136], glucuronoside transmembrane transporter activity [GO:0015164], glycerol-3-phosphate transmembrane transporter activity [GO:0015169], lipopolysaccharide transmembrane transporter activity [GO:0015221], ABC-type teichoic acid transporter activity [GO:0015438], glycerol-phosphate:phosphate antiporter activity [GO:0015527], N-acetylglucosamine transmembrane transporter activity [GO:0015572], methylgalactoside transmembrane transporter activity [GO:0015592], peptidoglycan transmembrane transporter activity [GO:0015647], nicotinamide mononucleotide transmembrane transporter activity [GO:0015663], galactosamine transmembrane transporter activity [GO:0019196], glucoside transmembrane transporter activity [GO:0042947], FMN transmembrane transporter activity [GO:0044610], sodium:galactoside symporter activity [GO:0044669], glycerone phosphate:phosphate antiporter activity [GO:0051407], GO:0051474, mannosylglycerate transmembrane transporter activity [GO:0051477], lysophospholipid:sodium symporter activity [GO:0051978], GO:0071917, glucosinolate transmembrane transporter activity [GO:0141165], ABC-type doxorubicin transporter activity [GO:1901242], 5-amino-1-ribofuranosylimidazole-4-carboxamide transmembrane transporter activity [GO:1903089] Also known as: carbohydrate derivative transporter activity Relationships: is a type of transmembrane transporter activity [GO:0022857]; is part of carbohydrate derivative transport [GO:1901264] Definition: Enables the transfer of carbohydrate derivative from one side of a membrane to the other.